{
  "gene_symbol": "NADK",
  "gene": "UniProtKB:O95544",
  "term_id": "GO:0003951",
  "gene_name": "NAD kinase",
  "term_label": "NAD+ kinase activity"
}